{
  "gene_name": "Disks large homolog 4",
  "term_label": "AMPA glutamate receptor clustering",
  "gene_symbol": "DLG4",
  "gene": "UniProtKB:P78352",
  "term_id": "GO:0097113"
}